{
  "gene_name": "SOSS complex subunit B1",
  "term_label": "DNA binding",
  "gene": "UniProtKB:Q9BQ15",
  "term_id": "GO:0003677",
  "gene_symbol": "NABP2"
}